{
  "gene_name": "Cancer_testis antigen family 45 member A9",
  "term_id": "UNKNOWN:0002",
  "term_label": "Unknown biological process",
  "gene_symbol": "CT45A9",
  "gene": "UniProtKB:P0DMV2"
}